carbamoyl phosphate metabolic process [GO:0070408] (BP) Sources: CHEBI:17672, GOC:mah, GOC:rph Definition: The chemical reactions and pathways involving carbamoyl phosphate, an intermediate in the urea cycle and other nitrogen compound metabolic pathways. Subtypes: carbamoyl phosphate biosynthetic process [GO:0070409] Also known as: carbamoyl phosphate metabolism Relationships: is a type of phosphate-containing compound metabolic process [GO:0006796]; is a type of GO:0019637